{
  "gene": "UniProtKB:Q8NC74",
  "gene_name": "RBBP8 N-terminal-like protein",
  "term_id": "UNKNOWN:0001",
  "gene_symbol": "RBBP8NL",
  "term_label": "Unknown molecular function"
}